{
  "gene": "UniProtKB:Q9H6S3",
  "gene_name": "Epidermal growth factor receptor kinase substrate 8-like protein 2",
  "term_id": "GO:1900029",
  "term_label": "positive regulation of ruffle assembly",
  "gene_symbol": "EPS8L2"
}